{
  "term_id": "GO:0001227",
  "gene_symbol": "ZNF688",
  "gene": "UniProtKB:P0C7X2",
  "gene_name": "Zinc finger protein 688",
  "term_label": "DNA-binding transcription repressor activity, RNA polymerase II-specific"
}